taurine dehydrogenase activity [GO:0050323] (molecular function) References: PMID:15073291 Sources: RHEA:18709 Relationships: is a type of oxidoreductase activity, acting on the CH-NH2 group of donors [GO:0016638] Also known as: taurine:(acceptor) oxidoreductase (deaminating), taurine:acceptor oxidoreductase (deaminating) Definition: Catalysis of the reaction: A + H2O + taurine = AH(2) + NH4 + sulfoacetaldehyde.